{
  "term_id": "GO:0051131",
  "term_label": "chaperone-mediated protein complex assembly",
  "gene": "UniProtKB:Q53FP2",
  "gene_name": "Novel acetylcholine receptor chaperone",
  "gene_symbol": "TMEM35A"
}